{
  "gene_symbol": "IGHV3-64",
  "term_id": "GO:0016064",
  "gene_name": "Immunoglobulin heavy variable 3-64",
  "term_label": "immunoglobulin mediated immune response",
  "gene": "UniProtKB:A0A075B6Q5"
}